{
  "gene": "UniProtKB:P57768",
  "gene_name": "Sorting nexin-16",
  "term_label": "phosphatidylinositol binding",
  "term_id": "GO:0035091",
  "gene_symbol": "SNX16"
}